{
  "term_label": "neuron projection",
  "gene": "UniProtKB:Q9P232",
  "gene_symbol": "CNTN3",
  "term_id": "GO:0043005",
  "gene_name": "Contactin-3"
}